histamine uptake [GO:0051615] (biological process) Definition: The directed movement of histamine into a cell, typically presynaptic neurons or glial cells. Histamine is a physiologically active amine, found in plant and animal tissue and released from mast cells as part of an allergic reaction in humans. Sources: GOC:ai Also known as: histamine import Relationships: is_a neurotransmitter uptake [GO:0001504]; is a type of GO:0051608 Regulation: regulated by regulation of histamine uptake [GO:0051616]; negatively regulated by negative regulation of histamine uptake [GO:0051617]; RO_0002213 by positive regulation of histamine uptake [GO:0051618]